{
  "term_id": "UNKNOWN:0002",
  "gene_symbol": "C14orf178",
  "gene_name": "Uncharacterized protein C14orf178",
  "term_label": "Unknown biological process",
  "gene": "UniProtKB:Q8N769"
}